{
  "gene_name": "XIAP-associated factor 1",
  "gene_symbol": "XAF1",
  "term_label": "Unknown molecular function",
  "gene": "UniProtKB:Q6GPH4",
  "term_id": "UNKNOWN:0001"
}